superoxide-generating NAD(P)H oxidase activity [GO:0016175] (molecular function) Relationships: is a type of GO:0050664 Definition: Catalysis of the reaction: NAD(P)H + O2 = NAD(P)H + O2-. References: PMID:10806195 Sources: GOC:ai Subtypes: superoxide-generating NADH oxidase activity [GO:0106291], GO:0106292 Also known as: cytochrome B-245